{
  "gene_symbol": "TP63",
  "gene": "UniProtKB:Q9H3D4",
  "term_label": "intrinsic apoptotic signaling pathway in response to DNA damage by p53 class mediator",
  "gene_name": "Tumor protein 63",
  "term_id": "GO:0042771"
}